{
  "term_label": "stereocilium",
  "gene_symbol": "GRXCR1",
  "gene": "UniProtKB:A8MXD5",
  "term_id": "GO:0032420",
  "gene_name": "Glutaredoxin domain-containing cysteine-rich protein 1"
}